{
  "term_label": "mitochondrial fission",
  "term_id": "GO:0000266",
  "gene_name": "Ganglioside-induced differentiation-associated protein 1",
  "gene": "UniProtKB:Q8TB36",
  "gene_symbol": "GDAP1"
}